{
  "gene_name": "Ubiquitin conjugation factor E4 B",
  "gene": "UniProtKB:O95155",
  "term_label": "ubiquitin-ubiquitin ligase activity",
  "term_id": "GO:0034450",
  "gene_symbol": "UBE4B"
}